{
  "gene_name": "Short transient receptor potential channel 4-associated protein",
  "term_label": "Cul4A-RING E3 ubiquitin ligase complex",
  "gene_symbol": "TRPC4AP",
  "gene": "UniProtKB:Q8TEL6",
  "term_id": "GO:0031464"
}